male urethra development [GO:0061069] (biological process) Sources: GOC:dph Relationships: is a type of urethra development [GO:0061068] Definition: The progression of the male urethra over time from its initial formation to the mature structure. The male urethra is a renal system organ that carries urine from the bladder through the penis to outside the body.